{
  "gene_name": "Ribosomal protein uL24-like",
  "term_id": "GO:0003735",
  "gene": "UniProtKB:Q9UNX3",
  "gene_symbol": "RPL26L1",
  "term_label": "structural constituent of ribosome"
}